{
  "term_id": "GO:0055056",
  "gene_name": "Solute carrier family 2, facilitated glucose transporter member 8",
  "gene": "UniProtKB:Q9NY64",
  "gene_symbol": "SLC2A8",
  "term_label": "D-glucose transmembrane transporter activity"
}